molting cycle, collagen and cuticulin-based cuticle [GO:0018996] (biological process) Also known as: collagen and cuticulin-based cuticle molting cycle Definition: The periodic shedding of part or all of a collagen and cuticulin-based cuticle, which is then replaced by a new collagen and cuticulin-based cuticle. An example of this is found in the Nematode worm, Caenorhabditis elegans. Relationships: is a type of molting cycle [GO:0042303] Sources: GOC:jl, GOC:mtg_sensu